{
  "term_id": "GO:0006999",
  "gene": "UniProtKB:Q7Z3B4",
  "gene_symbol": "NUP54",
  "gene_name": "Nucleoporin p54",
  "term_label": "nuclear pore organization"
}